{
  "gene_symbol": "GATD1",
  "gene_name": "Glutamine amidotransferase-like class 1 domain-containing protein 1",
  "term_id": "GO:0019172",
  "term_label": "glyoxalase III activity",
  "gene": "UniProtKB:Q8NB37"
}